{
  "gene_name": "Serine_threonine-protein kinase RIO2",
  "gene_symbol": "RIOK2",
  "term_label": "nucleus",
  "gene": "UniProtKB:Q9BVS4",
  "term_id": "GO:0005634"
}